testosterone 6-beta-hydroxylase activity [GO:0050649] (molecular function) References: PMID:11726664 Sources: RHEA:46296 Also known as: testosterone 6b-hydroxylase activity Relationships: is a type of GO:0008395 Definition: Catalysis of the reaction: O2 + reduced [NADPH--hemoprotein reductase] + testosterone = 6beta,17beta-dihydroxyandrost-4-en-3-one + H+ + H2O + oxidized [NADPH--hemoprotein reductase].